negative regulation of inner ear receptor cell differentiation [GO:2000981] (BP) Also known as: negative regulation of inner ear hair cell differentiation Sources: GOC:obol Relationships: is a type of negative regulation of mechanoreceptor differentiation [GO:0045632]; is_a regulation of inner ear receptor cell differentiation [GO:2000980]; negatively regulates inner ear receptor cell differentiation [GO:0060113] Subtypes: negative regulation of inner ear auditory receptor cell differentiation [GO:0045608] Definition: Any process that stops, prevents or reduces the frequency, rate or extent of inner ear receptor cell differentiation.